{
  "term_label": "GTPase activator activity",
  "term_id": "GO:0005096",
  "gene_symbol": "STXBP5",
  "gene": "UniProtKB:Q5T5C0",
  "gene_name": "Syntaxin-binding protein 5"
}